{
  "term_id": "GO:0006357",
  "gene_symbol": "ZBTB9",
  "gene_name": "Zinc finger and BTB domain-containing protein 9",
  "gene": "UniProtKB:Q96C00",
  "term_label": "regulation of transcription by RNA polymerase II"
}